negative regulation of cilium movement [GO:0003354] (biological process) Definition: Any process that decreases the rate, frequency, or extent of cilium movement, the directed, self-propelled movement of a cilium. Sources: GOC:dph Also known as: negative regulation of microtubule-based flagellum movement, negative regulation of flagellum movement Note: Note that we deem cilium and microtubule-based flagellum to be equivalent. Relationships: is a type of regulation of cilium movement [GO:0003352]; is a type of GO:0048523; negatively regulates cilium movement [GO:0003341] Subtypes: negative regulation of flagellated sperm motility [GO:1901318]